positive regulation of response to drug [GO:2001025] (biological process) Subtypes: positive regulation of cellular response to drug [GO:2001040] Sources: GOC:obol Also known as: positive regulation of drug resistance, positive regulation of drug susceptibility/resistance Definition: Any process that activates or increases the frequency, rate or extent of response to drug. Relationships: is a type of positive regulation of response to stimulus [GO:0048584]; is a type of regulation of response to drug [GO:2001023]; positively regulates response to xenobiotic stimulus [GO:0009410]